{
  "term_id": "UNKNOWN:0003",
  "gene_name": "Putative uncharacterized protein C8orf44",
  "gene": "UniProtKB:Q96CB5",
  "gene_symbol": "C8orf44",
  "term_label": "Unknown cellular component"
}